{
  "gene": "UniProtKB:P10244",
  "gene_symbol": "MYBL2",
  "term_label": "nucleus",
  "term_id": "GO:0005634",
  "gene_name": "Myb-related protein B"
}